{
  "gene_name": "Rap1 GTPase-activating protein 2",
  "gene": "UniProtKB:Q684P5",
  "term_label": "plasma membrane",
  "term_id": "GO:0005886",
  "gene_symbol": "RAP1GAP2"
}